{
  "term_id": "UNKNOWN:0001",
  "gene": "UniProtKB:A4D1T9",
  "gene_symbol": "PRSS37",
  "gene_name": "Probable inactive serine protease 37",
  "term_label": "Unknown molecular function"
}